negative regulation of centriole elongation [GO:1903723] (biological process) Also known as: down regulation of centriole elongation, down-regulation of centriole elongation, downregulation of centriole elongation, inhibition of centriole elongation Relationships: is a type of negative regulation of cell cycle process [GO:0010948]; is a type of regulation of centriole elongation [GO:1903722]; negatively regulates GO:0061511 References: PMID:20616062 Sources: GOC:TermGenie, GOC:als, GO_REF:0000058 Definition: Any process that stops, prevents or reduces the frequency, rate or extent of centriole elongation.